serine-pyruvate aminotransferase complex [GO:0005969] (cellular component) Relationships: is a type of transferase complex [GO:1990234]; is part of cytoplasm [GO:0005737] References: PMID:22751661, PMID:851432 Also known as: serine-pyruvate aminotransferase, type 1 complex, serine-pyruvate aminotransferase, type 2B complex Definition: A protein homodimeric complex that catalyzes the formation of hydroxypyruvate and alanine from serine and pyruvate.